{
  "gene": "UniProtKB:Q00987",
  "gene_symbol": "MDM2",
  "term_id": "GO:0061630",
  "term_label": "ubiquitin protein ligase activity",
  "gene_name": "E3 ubiquitin-protein ligase Mdm2"
}